{
  "gene_symbol": "BRMS1",
  "gene_name": "Breast cancer metastasis-suppressor 1",
  "term_id": "GO:0000122",
  "gene": "UniProtKB:Q9HCU9",
  "term_label": "negative regulation of transcription by RNA polymerase II"
}